{
  "gene_name": "26S proteasome regulatory subunit 4",
  "gene_symbol": "PSMC1",
  "term_label": "proteasome regulatory particle, base subcomplex",
  "gene": "UniProtKB:P62191",
  "term_id": "GO:0008540"
}